{
  "gene": "UniProtKB:Q6IPT4",
  "gene_name": "NADH-cytochrome b5 reductase-like",
  "gene_symbol": "CYB5RL",
  "term_label": "oxidoreductase activity",
  "term_id": "GO:0016491"
}